{
  "gene": "UniProtKB:Q99879",
  "gene_name": "Histone H2B type 1-M",
  "gene_symbol": "H2BC14",
  "term_label": "chromatin organization",
  "term_id": "GO:0006325"
}